positive regulation of ferroptosis [GO:0160020] (biological process) Relationships: is a type of positive regulation of programmed cell death [GO:0043068]; is a type of GO:0110075; positively regulates ferroptosis [GO:0097707] References: PMID:32015325 Definition: Any process that activates or increases the frequency, rate or extent of ferroptosis.